auxin transport [GO:0060918] (biological process) Definition: The directed movement of auxin into, out of or within a cell, or between cells, by means of some agent such as a transporter or pore. Auxins are a group of plant hormones that regulates aspects of plant growth. Subtypes: auxin polar transport [GO:0009926], auxin export across the plasma membrane [GO:0010315], GO:0060919, GO:0080162 Sources: GOC:dph, GOC:tb Relationships: is a type of hormone transport [GO:0009914]